chloroplast photosystem II [GO:0030095] (cellular component) Definition: An integral chloroplast membrane complex containing the P680 reaction center. In the light, PSII functions as a water-plastoquinone oxidoreductase, transferring electrons from water to plastoquinone. Sources: GOC:jid, GOC:mtg_sensu Relationships: is_a GO:0009523; is a type of chloroplast thylakoid membrane protein complex [GO:0098807]